{
  "gene_symbol": "KRT1",
  "gene": "UniProtKB:P04264",
  "term_label": "structural constituent of skin epidermis",
  "term_id": "GO:0030280",
  "gene_name": "Keratin, type II cytoskeletal 1"
}